{
  "term_label": "innate immune response",
  "gene_name": "Defensin alpha 5",
  "gene": "UniProtKB:Q01523",
  "term_id": "GO:0045087",
  "gene_symbol": "DEFA5"
}